plasma membrane respiratory chain complex IV assembly [GO:0033618] (biological process) Relationships: is a type of respiratory chain complex IV assembly [GO:0008535]; is part of plasma membrane organization [GO:0007009] Also known as: plasma membrane cytochrome c oxidase biogenesis, plasma membrane cytochrome c oxidase complex assembly Sources: GOC:mah Definition: The aggregation, arrangement and bonding together of a set of components to form respiratory chain complex IV (also known as cytochrome c oxidase) in the plasma membrane.